{
  "gene": "UniProtKB:Q86U86",
  "term_label": "RSC-type complex",
  "gene_symbol": "PBRM1",
  "term_id": "GO:0016586",
  "gene_name": "Protein polybromo-1"
}